regulation of muscle cell apoptotic process [GO:0010660] (biological process) Relationships: is a type of regulation of apoptotic process [GO:0042981]; regulates muscle cell apoptotic process [GO:0010657] Sources: GOC:dph, GOC:mtg_apoptosis, GOC:tb Also known as: regulation of muscle cell apoptosis Subtypes: GO:0010656, GO:0010661, regulation of striated muscle cell apoptotic process [GO:0010662], regulation of smooth muscle cell apoptotic process [GO:0034391] Definition: Any process that modulates the rate or frequency of muscle cell apoptotic process, a form of programmed cell death induced by external or internal signals that trigger the activity of proteolytic caspases whose actions dismantle a muscle cell and result in its death.